regulation of T cell extravasation [GO:2000407] (biological process) Definition: Any process that modulates the frequency, rate or extent of T cell extravasation. Sources: GOC:mah Relationships: is a type of regulation of cellular extravasation [GO:0002691]; is_a GO:2000404; regulates GO:0072683 Also known as: regulation of T lymphocyte extravasation, regulation of T-cell extravasation, regulation of T-lymphocyte extravasation Subtypes: negative regulation of T cell extravasation [GO:2000408], positive regulation of T cell extravasation [GO:2000409], regulation of CD8-positive, alpha-beta T cell extravasation [GO:2000449]